{
  "gene": "UniProtKB:Q9H0X4",
  "gene_symbol": "FAM234A",
  "term_label": "Unknown biological process",
  "term_id": "UNKNOWN:0002",
  "gene_name": "Protein FAM234A"
}